{
  "term_label": "cell surface receptor protein tyrosine kinase signaling pathway",
  "gene_symbol": "YES1",
  "gene_name": "Tyrosine-protein kinase Yes",
  "term_id": "GO:0007169",
  "gene": "UniProtKB:P07947"
}